{
  "gene_symbol": "COX6B2",
  "gene_name": "Cytochrome c oxidase subunit 6B2",
  "term_id": "GO:0005739",
  "term_label": "mitochondrion",
  "gene": "UniProtKB:Q6YFQ2"
}